{
  "gene_symbol": "KRT40",
  "gene_name": "Keratin, type I cytoskeletal 40",
  "term_id": "GO:0030280",
  "term_label": "structural constituent of skin epidermis",
  "gene": "UniProtKB:Q6A162"
}